{
  "term_label": "negative regulation of apoptotic process",
  "term_id": "GO:0043066",
  "gene": "UniProtKB:P04626",
  "gene_name": "Receptor tyrosine-protein kinase erbB-2",
  "gene_symbol": "ERBB2"
}